norepinephrine catabolic process [GO:0042422] (BP) Relationships: is a type of GO:0042415; is a type of catecholamine catabolic process [GO:0042424] Sources: GOC:jl, ISBN:0198506732 Also known as: levarterenol catabolic process, levarterenol catabolism, noradrenaline catabolic process, noradrenaline catabolism, norepinephrine breakdown, norepinephrine catabolism, norepinephrine degradation Definition: The chemical reactions and pathways resulting in the breakdown of norepinephrine, a hormone secreted by the adrenal medulla, and a neurotransmitter in the sympathetic peripheral nervous system and in some tracts in the central nervous system. It is also the demethylated biosynthetic precursor of epinephrine.